{
  "gene": "UniProtKB:Q13360",
  "term_id": "GO:0000981",
  "term_label": "DNA-binding transcription factor activity, RNA polymerase II-specific",
  "gene_name": "Zinc finger protein 177",
  "gene_symbol": "ZNF177"
}